protein deamination [GO:0018277] (biological process) Subtypes: N-terminal protein amino acid deamination, from amino carbon [GO:0018058] Definition: The removal of an amino group from a protein amino acid. Relationships: is a type of protein modification process [GO:0036211] Sources: GOC:ai Also known as: protein amino acid deamination